{
  "term_label": "regulation of gene expression",
  "gene_name": "Ret finger protein-like 4B",
  "gene_symbol": "RFPL4B",
  "gene": "UniProtKB:Q6ZWI9",
  "term_id": "GO:0010468"
}